{
  "gene_symbol": "CPSF4L",
  "gene_name": "Putative cleavage and polyadenylation specificity factor subunit 4-like protein",
  "term_id": "UNKNOWN:0002",
  "gene": "UniProtKB:A6NMK7",
  "term_label": "Unknown biological process"
}